cell proliferation in forebrain [GO:0021846] (biological process) Subtypes: subpallium cell proliferation in forebrain [GO:0022012], GO:0022013 Sources: GOC:cls, GOC:dgh, GOC:dph, GOC:jid, GO_REF:0000021 Definition: The creation of greater cell numbers in the forebrain due to cell division of progenitor cells. Relationships: is a type of neural precursor cell proliferation [GO:0061351]; is part of forebrain development [GO:0030900]